bile acid biosynthetic process [GO:0006699] (BP) Relationships: is a type of bile acid metabolic process [GO:0008206]; is_a GO:0072330 Also known as: bile acid anabolism, bile acid biosynthesis, bile acid formation, bile acid synthesis Definition: The chemical reactions and pathways resulting in the formation of bile acids, any of a group of steroid carboxylic acids occurring in bile. Regulation: regulated by regulation of bile acid biosynthetic process [GO:0070857]; negatively regulated by GO:0070858; positively regulated by GO:0070859 Sources: GOC:go_curators